{
  "gene_name": "Keratin, type II cuticular Hb3",
  "gene": "UniProtKB:P78385",
  "gene_symbol": "KRT83",
  "term_id": "GO:0045109",
  "term_label": "intermediate filament organization"
}